{
  "gene": "UniProtKB:O75962",
  "gene_name": "Triple functional domain protein",
  "gene_symbol": "TRIO",
  "term_label": "axon guidance",
  "term_id": "GO:0007411"
}